{
  "gene_symbol": "SLC25A21",
  "gene_name": "Mitochondrial 2-oxodicarboxylate carrier",
  "term_id": "UNKNOWN:0002",
  "term_label": "Unknown biological process",
  "gene": "UniProtKB:Q9BQT8"
}